{
  "term_id": "GO:0000981",
  "gene_symbol": "GATAD2A",
  "gene": "UniProtKB:Q86YP4",
  "gene_name": "Transcriptional repressor p66-alpha",
  "term_label": "DNA-binding transcription factor activity, RNA polymerase II-specific"
}